seryl-tRNA aminoacylation [GO:0006434] (biological process) Definition: The process of coupling serine to seryl-tRNA, catalyzed by seryl-tRNA synthetase. The seryl-tRNA synthetase is a class-II synthetase. The activated amino acid is transferred to the 3'-OH group of a serine-accetping tRNA. Sources: GOC:mcc, ISBN:0716730510 Subtypes: mitochondrial seryl-tRNA aminoacylation [GO:0070158] Relationships: is a type of tRNA aminoacylation for protein translation [GO:0006418]; has part GO:0001717